{
  "term_id": "GO:0009100",
  "gene_symbol": "OGA",
  "term_label": "glycoprotein metabolic process",
  "gene_name": "Protein O-GlcNAcase",
  "gene": "UniProtKB:O60502"
}